{
  "term_label": "microtubule nucleation",
  "term_id": "GO:0007020",
  "gene_name": "Gamma-tubulin complex component 4",
  "gene": "UniProtKB:Q9UGJ1",
  "gene_symbol": "TUBGCP4"
}